{
  "term_id": "GO:0006511",
  "gene": "UniProtKB:Q68DV7",
  "gene_symbol": "RNF43",
  "term_label": "ubiquitin-dependent protein catabolic process",
  "gene_name": "E3 ubiquitin-protein ligase RNF43"
}